{
  "gene_symbol": "PMS2P1",
  "term_id": "UNKNOWN:0003",
  "gene": "UniProtKB:A4D2B8",
  "term_label": "Unknown cellular component",
  "gene_name": "Putative postmeiotic segregation increased 2-like protein 1"
}